{
  "gene_symbol": "ZNF454",
  "gene": "UniProtKB:Q8N9F8",
  "term_id": "GO:0006357",
  "gene_name": "Zinc finger protein 454",
  "term_label": "regulation of transcription by RNA polymerase II"
}